{
  "gene_symbol": "CPVL",
  "gene_name": "Probable serine carboxypeptidase CPVL",
  "term_label": "Unknown cellular component",
  "gene": "UniProtKB:Q9H3G5",
  "term_id": "UNKNOWN:0003"
}